{
  "term_label": "immunoglobulin mediated immune response",
  "gene_name": "Immunoglobulin heavy variable 1_OR15-1 (non-functional) (Fragment)",
  "gene": "UniProtKB:A0A075B7D0",
  "gene_symbol": "IGHV1OR15-1",
  "term_id": "GO:0016064"
}